{
  "gene_name": "CUB domain-containing protein",
  "term_label": "Unknown biological process",
  "gene_symbol": "SPADH",
  "gene": "UniProtKB:A0A494C103",
  "term_id": "UNKNOWN:0002"
}